{
  "gene": "UniProtKB:Q8NA82",
  "gene_name": "Probable E3 ubiquitin-protein ligase MARCHF10",
  "term_label": "Unknown cellular component",
  "gene_symbol": "MARCHF10",
  "term_id": "UNKNOWN:0003"
}